cardiac ventricle development [GO:0003231] (biological process) Regulation: regulated by regulation of cardiac ventricle development [GO:1904412]; negatively regulated by negative regulation of cardiac ventricle development [GO:1904413]; positively regulated by positive regulation of cardiac ventricle development [GO:1904414] Sources: GOC:mtg_heart Definition: The process whose specific outcome is the progression of a cardiac ventricle over time, from its formation to the mature structure. A cardiac ventricle receives blood from a cardiac atrium and pumps it out of the heart. Relationships: is_a cardiac chamber development [GO:0003205]